lysozyme activity [GO:0003796] (molecular function) Also known as: 1,4-N-acetylmuramidase activity, N,O-diacetylmuramidase activity, mucopeptide N-acetylmuramoylhydrolase activity, mucopeptide glucohydrolase activity, muramidase activity, L-7001, PR1-lysozyme, globulin G, globulin G1, lysozyme g, peptidoglycan N-acetylmuramoylhydrolase activity Regulation: negatively regulated by lysozyme inhibitor activity [GO:0060241]; positively regulated by GO:1903592 References: PMID:22748813 Sources: EC:3.2.1.17 Relationships: is a type of GO:0004553; is a type of GO:0061783 Definition: Catalysis of the hydrolysis of the beta-(1->4) linkages between N-acetylmuramic acid and N-acetyl-D-glucosamine residues in a peptidoglycan.